{
  "term_id": "GO:0005886",
  "gene": "UniProtKB:Q9BZZ2",
  "term_label": "plasma membrane",
  "gene_symbol": "SIGLEC1",
  "gene_name": "Sialoadhesin"
}